septation initiation signaling [GO:0031028] (biological process) Relationships: is a type of small GTPase-mediated signal transduction [GO:0007264] Definition: The series of molecular signals, mediated by the small GTPase Ras, that results in the initiation of contraction of the contractile ring, at the beginning of cytokinesis and cell division by septum formation. The pathway coordinates chromosome segregation with mitotic exit and cytokinesis. Also known as: SIN, septation initiation network, septation initiation signalling, septation initiation signaling cascade References: PMID:16775007 Sources: GOC:mah, GOC:vw Regulation: regulated by GO:0031029; negatively regulated by negative regulation of septation initiation signaling [GO:0031030]; positively regulated by positive regulation of septation initiation signaling [GO:0031031]